{
  "gene_name": "Ashwin",
  "gene_symbol": "C2orf49",
  "term_label": "Unknown molecular function",
  "gene": "UniProtKB:Q9BVC5",
  "term_id": "UNKNOWN:0001"
}